chlorophyll a biosynthetic process [GO:0033305] (biological process) Relationships: is a type of chlorophyll biosynthetic process [GO:0015995] Also known as: chlorophyll a anabolism, chlorophyll a biosynthesis, chlorophyll a formation, chlorophyll a synthesis Sources: GOC:mah Subtypes: chlorophyll a biosynthetic process via phytyl diphosphate [GO:0033311], GO:0033312 Definition: The chemical reactions and pathways leading to the formation of chlorophyll a.